{
  "term_label": "piRNA processing",
  "gene": "UniProtKB:Q9Y2W6",
  "term_id": "GO:0034587",
  "gene_symbol": "TDRKH",
  "gene_name": "Tudor and KH domain-containing protein"
}